{
  "gene": "UniProtKB:P31269",
  "term_label": "proximal/distal pattern formation",
  "gene_name": "Homeobox protein Hox-A9",
  "term_id": "GO:0009954",
  "gene_symbol": "HOXA9"
}